{
  "gene_name": "Zinc finger protein 737",
  "term_label": "RNA polymerase II cis-regulatory region sequence-specific DNA binding",
  "term_id": "GO:0000978",
  "gene_symbol": "ZNF737",
  "gene": "UniProtKB:O75373"
}